{
  "gene_name": "Small proline-rich protein 2F",
  "term_id": "UNKNOWN:0002",
  "gene": "UniProtKB:Q96RM1",
  "term_label": "Unknown biological process",
  "gene_symbol": "SPRR2F"
}